detection of electrical stimulus [GO:0050981] (biological process) Subtypes: detection of electrical stimulus involved in regulation of muscle adaptation [GO:0014879], detection of electrical stimulus involved in sensory perception [GO:0050963] Sources: GOC:ai, GOC:dos Definition: The series of events by which an electrical stimulus is received and converted into a molecular signal. Relationships: is a type of GO:0009582; is_a GO:0051602